{
  "gene_symbol": "PRAMEF6",
  "gene_name": "PRAME family member 6",
  "term_id": "GO:1990756",
  "term_label": "ubiquitin-like ligase-substrate adaptor activity",
  "gene": "UniProtKB:Q5VXH4"
}